{
  "term_label": "rRNA processing",
  "gene_symbol": "DDX49",
  "gene": "UniProtKB:Q9Y6V7",
  "gene_name": "Probable ATP-dependent RNA helicase DDX49",
  "term_id": "GO:0006364"
}